nail development [GO:0035878] (biological process) Definition: The process whose specific outcome is the progression of a nail over time, from its formation to the mature structure. A nail is a horn-like envelope covering the outer end of a finger or toe, and consists of the nail plate, the nail matrix and the nail bed below it, and the grooves surrounding it. Sources: GOC:bf, ISBN:0323025781, UBERON:0001705, Wikipedia:Nail_(anatomy) Relationships: is a type of anatomical structure development [GO:0048856]; is part of limb development [GO:0060173]